{
  "gene_symbol": "KCNE1",
  "term_label": "transmembrane transporter binding",
  "gene_name": "Potassium voltage-gated channel subfamily E member 1",
  "term_id": "GO:0044325",
  "gene": "UniProtKB:P15382"
}